protein-phosphatidylethanolamide deconjugating activity [GO:0019786] (molecular function) Definition: Catalysis of the reaction: [protein]-C-terminal L-amino acid-glycyl-phosphatidylethanolamide + H2O = [protein]-C-terminal L-amino acid-glycine + a 1,2-diacyl-sn-glycero-3-phosphoethanolamine. An example of this reaction is the removal of ATG8 from membranes to which it is covalently linked to a phosphatidylethanolamid via its terminal glycine residue. References: PMID:22240591, PMID:22652539, PMID:28330855, PMID:2882172, PMID:28901328 Also known as: Atg8-specific protease activity, APG8-specific protease activity, ATG8-PE deconjugation activity, ATG8-PE hydrolase activity, Atg8-specific peptidase activity, APG8-PE hydrolase Relationships: is a type of hydrolase activity [GO:0016787]; is_a GO:0140096